{
  "gene_name": "Squalene synthase",
  "gene_symbol": "FDFT1",
  "gene": "UniProtKB:P37268",
  "term_label": "squalene synthase [NAD(P)H] activity",
  "term_id": "GO:0051996"
}